fucokinase activity [GO:0050201] (molecular function) Sources: EC:2.7.1.52, RHEA:13241 Relationships: is a type of GO:0016301; is a type of GO:0016773 Definition: Catalysis of the reaction: L-fucose + ATP = beta-L-fucose 1-phosphate + ADP + 2 H+. Also known as: ATP:6-deoxy-L-galactose 1-phosphotransferase activity, ATP:beta-L-fucose 1-phosphotransferase activity, L-fucokinase activity, L-fucose kinase activity, fucokinase (phosphorylating) activity, fucose kinase activity